protein depropionylation [GO:0106230] (biological process) Definition: The removal of a propionyl group from a residue in a peptide or protein. References: PMID:30026585 Sources: GOC:sp Relationships: is a type of protein deacylation [GO:0035601]